sulfite transmembrane transport [GO:0000316] (biological process) Regulation: regulated by regulation of sulfite transmembrane transport [GO:1900071]; positively regulated by positive regulation of sulfite transmembrane transport [GO:1900072] Definition: The directed movement of sulfite into, out of or within a cell, or between cells, by means of some agent such as a transporter or pore. Sources: GOC:krc Relationships: is_a inorganic anion transport [GO:0015698]; is a type of GO:0055085; is_a sulfur compound transport [GO:0072348] Subtypes: GO:0160244 Also known as: sulphite transport